cyclic nucleotide transport [GO:0070729] (biological process) Relationships: is a type of nucleotide transport [GO:0006862] Definition: The directed movement of a cyclic nucleotide, any nucleotide in which phosphate group is in diester linkage to two positions on the sugar residue, into, out of or within a cell. Sources: GOC:mah, ISBN:0198506732 Subtypes: cAMP transport [GO:0070730], cGMP transport [GO:0070731], cyclic-GMP-AMP transmembrane import across plasma membrane [GO:0140361]